{
  "gene_symbol": "BARHL1",
  "gene_name": "BarH-like 1 homeobox protein",
  "term_id": "GO:0005634",
  "term_label": "nucleus",
  "gene": "UniProtKB:Q9BZE3"
}